{
  "term_label": "synapse organization",
  "gene_name": "SH3 and multiple ankyrin repeat domains protein 1",
  "term_id": "GO:0050808",
  "gene": "UniProtKB:Q9Y566",
  "gene_symbol": "SHANK1"
}